{
  "gene": "UniProtKB:Q8IZ08",
  "term_id": "GO:0004930",
  "gene_symbol": "GPR135",
  "term_label": "G protein-coupled receptor activity",
  "gene_name": "G-protein coupled receptor 135"
}